{
  "term_id": "UNKNOWN:0001",
  "gene": "UniProtKB:Q96BI1",
  "term_label": "Unknown molecular function",
  "gene_name": "Solute carrier family 22 member 18",
  "gene_symbol": "SLC22A18"
}